{
  "gene_name": "Transcription termination factor 3, mitochondrial",
  "term_id": "GO:1903108",
  "gene": "UniProtKB:Q96E29",
  "term_label": "regulation of mitochondrial transcription",
  "gene_symbol": "MTERF3"
}